{
  "gene": "UniProtKB:Q9NS56",
  "gene_symbol": "TOPORS",
  "term_id": "GO:0036064",
  "gene_name": "E3 ubiquitin-protein ligase Topors",
  "term_label": "ciliary basal body"
}